{
  "gene_name": "Transmembrane protein 252",
  "term_id": "UNKNOWN:0002",
  "term_label": "Unknown biological process",
  "gene_symbol": "TMEM252",
  "gene": "UniProtKB:Q8N6L7"
}